{
  "gene_symbol": "RUNX1",
  "term_id": "GO:0045595",
  "gene": "UniProtKB:Q01196",
  "term_label": "regulation of cell differentiation",
  "gene_name": "Runt-related transcription factor 1"
}